{
  "gene_name": "Uncharacterized protein C8orf74",
  "term_label": "Unknown molecular function",
  "gene": "UniProtKB:Q6P047",
  "gene_symbol": "C8orf74",
  "term_id": "UNKNOWN:0001"
}